{
  "gene_name": "Coiled-coil domain-containing protein 178",
  "gene": "UniProtKB:Q5BJE1",
  "term_id": "UNKNOWN:0002",
  "gene_symbol": "CCDC178",
  "term_label": "Unknown biological process"
}